{
  "gene": "UniProtKB:O43474",
  "term_id": "GO:0000978",
  "gene_symbol": "KLF4",
  "gene_name": "Krueppel-like factor 4",
  "term_label": "RNA polymerase II cis-regulatory region sequence-specific DNA binding"
}